{
  "term_label": "protein serine/threonine kinase activity",
  "gene_symbol": "TSSK2",
  "gene": "UniProtKB:Q96PF2",
  "gene_name": "Testis-specific serine_threonine-protein kinase 2",
  "term_id": "GO:0004674"
}